{
  "term_label": "NAD+ poly-ADP-ribosyltransferase activity",
  "term_id": "GO:0003950",
  "gene_name": "Ecto-ADP-ribosyltransferase 5",
  "gene_symbol": "ART5",
  "gene": "UniProtKB:Q96L15"
}